{
  "term_id": "GO:0019509",
  "gene_symbol": "MTAP",
  "gene_name": "S-methyl-5'-thioadenosine phosphorylase",
  "gene": "UniProtKB:Q13126",
  "term_label": "L-methionine salvage from methylthioadenosine"
}